{
  "term_id": "GO:1903457",
  "gene_symbol": "LDHD",
  "term_label": "lactate catabolic process",
  "gene_name": "Probable D-lactate dehydrogenase, mitochondrial",
  "gene": "UniProtKB:Q86WU2"
}